{
  "term_id": "GO:0005737",
  "gene_name": "Myosin light chain kinase family member 4",
  "gene": "UniProtKB:Q86YV6",
  "gene_symbol": "MYLK4",
  "term_label": "cytoplasm"
}